{
  "gene_name": "Pyruvate dehydrogenase phosphatase regulatory subunit, mitochondrial",
  "term_id": "GO:0005737",
  "term_label": "cytoplasm",
  "gene_symbol": "PDPR",
  "gene": "UniProtKB:Q8NCN5"
}